detection of steroid hormone stimulus [GO:0051467] (biological process) Subtypes: detection of glucocorticoid hormone stimulus [GO:0051468] Relationships: is a type of detection of hormone stimulus [GO:0009720]; is a type of response to steroid hormone [GO:0048545] Definition: The series of events by which a steroid hormone stimulus is received by a cell and converted into a molecular signal. Sources: GOC:ai